{
  "gene_symbol": "ACAA2",
  "gene_name": "3-ketoacyl-CoA thiolase, mitochondrial",
  "term_label": "mitochondrion",
  "gene": "UniProtKB:P42765",
  "term_id": "GO:0005739"
}